{
  "term_id": "GO:0000776",
  "term_label": "kinetochore",
  "gene": "UniProtKB:O60566",
  "gene_name": "Mitotic checkpoint serine_threonine-protein kinase BUB1 beta",
  "gene_symbol": "BUB1B"
}